{
  "gene": "UniProtKB:Q495T6",
  "term_id": "GO:0016485",
  "term_label": "protein processing",
  "gene_name": "Membrane metallo-endopeptidase-like 1",
  "gene_symbol": "MMEL1"
}